{
  "term_id": "GO:0005829",
  "gene": "UniProtKB:Q7RTZ2",
  "gene_name": "Ubiquitin carboxyl-terminal hydrolase 17-like protein 1",
  "term_label": "cytosol",
  "gene_symbol": "USP17L1"
}